{
  "gene": "UniProtKB:Q6ZP65",
  "term_label": "Unknown cellular component",
  "gene_name": "BICD family-like cargo adapter 1",
  "term_id": "UNKNOWN:0003",
  "gene_symbol": "BICDL1"
}